cortical layer of collagen and cuticulin-based cuticle extracellular matrix [GO:0060106] (cellular component) Relationships: is_a cellular anatomical structure [GO:0110165]; is part of cuticular extracellular matrix [GO:0060102] Definition: The cuticle layer that lies directly beneath the lipid-containing epicuticle. The cortical layer contains collagens and insoluble, non-collagenous cuticulins and is characterized by a distinct annular pattern consisting of regularly spaced annular ridges delineated by annular furrows. An example of this component is found in Caenorhabditis elegans. Sources: GOC:dph, GOC:kmv, ISSN:15518507